{
  "gene_symbol": "HADHA",
  "term_label": "fatty acid beta-oxidation",
  "gene": "UniProtKB:P40939",
  "term_id": "GO:0006635",
  "gene_name": "Trifunctional enzyme subunit alpha, mitochondrial"
}